{
  "gene": "UniProtKB:P06727",
  "term_id": "GO:0005543",
  "term_label": "phospholipid binding",
  "gene_symbol": "APOA4",
  "gene_name": "Apolipoprotein A-IV"
}